{
  "gene_symbol": "SUSD1",
  "gene": "UniProtKB:Q6UWL2",
  "term_id": "UNKNOWN:0002",
  "gene_name": "Sushi domain-containing protein 1",
  "term_label": "Unknown biological process"
}